{
  "gene_name": "Derlin-2",
  "gene": "UniProtKB:Q9GZP9",
  "term_label": "endoplasmic reticulum membrane",
  "gene_symbol": "DERL2",
  "term_id": "GO:0005789"
}